{
  "gene_symbol": "SNRPD2",
  "gene": "UniProtKB:P62316",
  "term_label": "Unknown molecular function",
  "gene_name": "Small nuclear ribonucleoprotein Sm D2",
  "term_id": "UNKNOWN:0001"
}